protein C inhibitor-coagulation factor XI complex [GO:0097183] (cellular component) Relationships: is a type of serine protease inhibitor complex [GO:0097180] References: PMID:2844223 Sources: GOC:ans Also known as: PCI-coagulation factor XI complex, SERPINA5-coagulation factor XI complex, plasma serine protease inhibitor-coagulation factor XI complex, protein C inhibitor-F11 complex, serpin A5-coagulation factor XI complex Definition: A heterodimeric protein complex that contains protein C inhibitor (SERPINA5) and coagulation factor XI (F11); formation of the complex inhibits the serine protease activity of coagulation factor XI.